ribose 1-dehydrogenase (NADP+) activity [GO:0050259] (molecular function) Relationships: is a type of oxidoreductase activity, acting on the CH-OH group of donors, NAD or NADP as acceptor [GO:0016616] Definition: Catalysis of the reaction: H2O + NADP+ + ribofuranose = D-ribonate + 2 H+ + NADPH. Also known as: D-ribose dehydrogenase (NADP+), D-ribose:NADP+ 1-oxidoreductase activity, NADP-pentose-dehydrogenase activity Sources: EC:1.1.1.115, RHEA:11676